{
  "gene_symbol": "MCAT",
  "gene": "UniProtKB:Q8IVS2",
  "term_id": "GO:0004314",
  "term_label": "[acyl-carrier-protein] S-malonyltransferase activity",
  "gene_name": "Malonyl-CoA-acyl carrier protein transacylase, mitochondrial"
}